symbiont-mediated suppression of host gene expression [GO:0039657] (biological process) Definition: A process in which a symbiont inhibits or disrupts expression of genes in its host. Gene expression is the process in which a gene's coding sequence is converted into a mature gene product or products (proteins or RNA). This includes the production of an RNA transcript as well as any processing to produce a mature RNA product or an mRNA (for protein-coding genes) and the translation of that mRNA into protein. Some protein processing events may be included when they are required to form an active form of a product from an inactive precursor form. The host is defined as the larger of the organisms involved in a symbiotic interaction. Relationships: is a type of symbiont-mediated perturbation of host gene expression [GO:0039656] Also known as: host gene expression shutoff, host gene expression shutoff by virus, suppression by virus of host gene expression Subtypes: symbiont-mediated suppression of host mRNA export from nucleus [GO:0039522] Sources: VZ:1582